{
  "term_label": "choline:sodium symporter activity",
  "term_id": "GO:0005307",
  "gene": "UniProtKB:Q9GZV3",
  "gene_symbol": "SLC5A7",
  "gene_name": "High affinity choline transporter 1"
}